{
  "term_id": "GO:0006357",
  "gene": "UniProtKB:Q6AZW8",
  "term_label": "regulation of transcription by RNA polymerase II",
  "gene_symbol": "ZNF660",
  "gene_name": "Zinc finger protein 660"
}